{
  "gene_symbol": "PTPRO",
  "term_label": "negative regulation of canonical Wnt signaling pathway",
  "term_id": "GO:0090090",
  "gene": "UniProtKB:Q16827",
  "gene_name": "Receptor-type tyrosine-protein phosphatase O"
}